{
  "gene_name": "Putative uncharacterized protein FLJ32790",
  "gene": "UniProtKB:Q96M66",
  "gene_symbol": "Q96M66",
  "term_id": "UNKNOWN:0002",
  "term_label": "Unknown biological process"
}